{
  "term_label": "regulation of DNA-templated transcription",
  "gene_name": "Zinc finger protein 141",
  "gene_symbol": "ZNF141",
  "gene": "UniProtKB:Q15928",
  "term_id": "GO:0006355"
}